{
  "gene": "UniProtKB:Q8N6U2",
  "term_id": "UNKNOWN:0001",
  "gene_name": "Putative uncharacterized protein encoded by LINC00612",
  "term_label": "Unknown molecular function",
  "gene_symbol": "LINC00612"
}